inner ear receptor cell differentiation involved in inner ear sensory epithelium regeneration [GO:0070660] (biological process) Relationships: is a type of inner ear receptor cell differentiation [GO:0060113]; is a type of mechanoreceptor differentiation involved in mechanosensory epithelium regeneration [GO:0070656]; is part of inner ear sensory epithelium regeneration [GO:0070659] Definition: Differentiation of new inner ear sensory hair cells to replace those lost or destroyed by injury. References: PMID:19381250 Sources: GOC:dsf